anterograde dendritic transport of messenger ribonucleoprotein complex [GO:0098964] (BP) Relationships: is a type of anterograde dendritic transport [GO:0098937] Also known as: anterograde dendritic transport of mRNA RNP complex Definition: The directed movement of a messenger ribonucleoprotein complex along microtubules in nerve cell dendrites towards the postsynapse. Sources: GOC:dos